cnida [GO:0140022] (cellular component) Also known as: cnidae (plural) Relationships: is a type of cellular anatomical structure [GO:0110165] Definition: A giant secretory organelle that comprises a bulb-shape capsule containing a coiled hollow tubule structure attached to it. A cnida defines the phylum Cnidaria. Sources: Wikipedia:Cnida#Structure_and_function